{
  "term_label": "nucleus",
  "gene_symbol": "PARP15",
  "gene_name": "Protein mono-ADP-ribosyltransferase PARP15",
  "gene": "UniProtKB:Q460N3",
  "term_id": "GO:0005634"
}